negative regulation of axial mesodermal cell fate specification [GO:0048329] (biological process) Definition: Any process that stops, prevents, or reduces the frequency, rate or extent of axial mesoderm cell fate specification. Sources: GOC:dgh Relationships: is a type of GO:0042662; is a type of regulation of axial mesodermal cell fate specification [GO:0048328]; negatively regulates axial mesodermal cell fate specification [GO:0048327] Also known as: down regulation of axial mesodermal cell fate specification, down-regulation of axial mesodermal cell fate specification, downregulation of axial mesodermal cell fate specification, inhibition of axial mesodermal cell fate specification